{
  "term_id": "GO:0004984",
  "term_label": "olfactory receptor activity",
  "gene_symbol": "OR6C3",
  "gene": "UniProtKB:Q9NZP0",
  "gene_name": "Olfactory receptor 6C3"
}